{
  "gene_symbol": "FAM111B",
  "term_label": "nucleus",
  "gene_name": "Serine protease FAM111B",
  "term_id": "GO:0005634",
  "gene": "UniProtKB:Q6SJ93"
}